{
  "gene_symbol": "YWHAH-AS1",
  "term_label": "Unknown cellular component",
  "term_id": "UNKNOWN:0003",
  "gene": "UniProtKB:Q9Y442",
  "gene_name": "Putative uncharacterized protein YWHAH-AS1"
}